{
  "gene_name": "Transmembrane domain-containing protein TMIGD3",
  "gene": "UniProtKB:P0DMS9",
  "gene_symbol": "TMIGD3",
  "term_id": "GO:0004888",
  "term_label": "transmembrane signaling receptor activity"
}